germ-line cyst encapsulation [GO:0048138] (biological process) Subtypes: GO:0048139, male germ-line cyst encapsulation [GO:0048140] Relationships: is a type of developmental process involved in reproduction [GO:0003006]; is a type of anatomical structure development [GO:0048856]; is part of GO:0007276; is part of morphogenesis of follicular epithelium [GO:0016333] Sources: GOC:jid Definition: Formation of a single follicular epithelium around the germ-line derived cells of a cyst.